{
  "gene_symbol": "DUXB",
  "gene_name": "Double homeobox protein B",
  "gene": "UniProtKB:A0A1W2PPF3",
  "term_label": "RNA polymerase II transcription regulatory region sequence-specific DNA binding",
  "term_id": "GO:0000977"
}